{
  "gene_name": "Protein scribble homolog",
  "term_label": "postsynaptic density",
  "gene_symbol": "SCRIB",
  "term_id": "GO:0014069",
  "gene": "UniProtKB:Q14160"
}